{
  "term_label": "Unknown molecular function",
  "gene_symbol": "ADCK2",
  "term_id": "UNKNOWN:0001",
  "gene": "UniProtKB:Q7Z695",
  "gene_name": "Uncharacterized aarF domain-containing protein kinase 2"
}